{
  "term_id": "GO:0016020",
  "gene_symbol": "SLC45A3",
  "gene": "UniProtKB:Q96JT2",
  "gene_name": "Solute carrier family 45 member 3",
  "term_label": "membrane"
}